{
  "gene": "UniProtKB:Q92556",
  "gene_symbol": "ELMO1",
  "gene_name": "Engulfment and cell motility protein 1",
  "term_label": "cell motility",
  "term_id": "GO:0048870"
}